{
  "gene": "UniProtKB:Q6ZSZ5",
  "term_id": "GO:0005886",
  "term_label": "plasma membrane",
  "gene_name": "Rho guanine nucleotide exchange factor 18",
  "gene_symbol": "ARHGEF18"
}